{
  "term_id": "GO:0090166",
  "gene": "UniProtKB:Q9H4B4",
  "gene_name": "Serine_threonine-protein kinase PLK3",
  "gene_symbol": "PLK3",
  "term_label": "Golgi disassembly"
}